{
  "gene": "UniProtKB:Q9BRR3",
  "gene_name": "Post-GPI attachment to proteins factor 4",
  "term_id": "GO:0000139",
  "gene_symbol": "PGAP4",
  "term_label": "Golgi membrane"
}